growth hormone receptor signaling pathway [GO:0060396] (biological process) Relationships: is a type of cell surface receptor protein tyrosine kinase signaling pathway [GO:0007169]; BFO_0000050 cellular response to growth hormone stimulus [GO:0071378] Regulation: RO_0002211 by regulation of growth hormone receptor signaling pathway [GO:0060398]; positively regulated by positive regulation of growth hormone receptor signaling pathway [GO:0060399]; negatively regulated by negative regulation of growth hormone receptor signaling pathway [GO:0060400] References: PMID:11445442 Sources: GOC:BHF, GOC:dph Definition: The series of molecular signals generated as a consequence of growth hormone receptor binding to its physiological ligand. Also known as: growth hormone receptor signalling pathway, GH receptor signaling pathway, cellular response to growth hormone Subtypes: growth hormone receptor signaling pathway via JAK-STAT [GO:0060397]